{
  "term_id": "GO:0055085",
  "gene_name": "Choline transporter-like protein 1",
  "term_label": "transmembrane transport",
  "gene": "UniProtKB:Q8WWI5",
  "gene_symbol": "SLC44A1"
}